{
  "gene_symbol": "ANXA11",
  "gene_name": "Annexin A11",
  "term_label": "phosphatidylserine binding",
  "term_id": "GO:0001786",
  "gene": "UniProtKB:P50995"
}